{
  "term_label": "Unknown biological process",
  "gene_symbol": "SPATA31D3",
  "term_id": "UNKNOWN:0002",
  "gene": "UniProtKB:P0C874",
  "gene_name": "Spermatogenesis-associated protein 31D3"
}